{
  "term_label": "plasma membrane",
  "gene_symbol": "SLC1A6",
  "term_id": "GO:0005886",
  "gene": "UniProtKB:P48664",
  "gene_name": "Excitatory amino acid transporter 4"
}